{
  "gene_name": "DNA primase large subunit",
  "term_id": "GO:0006270",
  "gene_symbol": "PRIM2",
  "gene": "UniProtKB:P49643",
  "term_label": "DNA replication initiation"
}